symbiont-mediated activation of host induced systemic resistance [GO:0052103] (biological process) References: PMID:31516360 Sources: GOC:mtg_pamgo_17jul06 Also known as: induction by organism of induced systemic resistance in other organism involved in symbiotic interaction, positive regulation by organism of induced systemic resistance in other organism involved in symbiotic interaction, activation by organism of ISR in host, activation by organism of induced systemic resistance in host, induction by organism of ISR in host, induction by symbiont of host induced systemic resistance, induction by symbiont of induced systemic resistance in host, induction of host induced systemic resistance, activation by symbiont of induced systemic resistance in host, stimulation by symbiont of induced systemic resistance in host, positive regulation by symbiont of host induced systemic resistance, positive regulation by symbiont of induced systemic resistance in host, up regulation by symbiont of induced systemic resistance in host, up-regulation by symbiont of induced systemic resistance in host, upregulation by symbiont of induced systemic resistance in host Definition: Any process in which a symbiont activates, maintains or increases the frequency, rate or extent of induced systemic resistance in the host organism; induced systemic resistance is a response that confers broad spectrum systemic resistance to disease and that does not depend upon salicylic acid signaling. The host is defined as the larger of the organisms involved in a symbiotic interaction. Relationships: is a type of symbiont-mediated perturbation of host induced systemic resistance [GO:0052159]